negative regulation of tRNA metabolic process [GO:1903327] (BP) Relationships: is a type of GO:0051253; is a type of regulation of tRNA metabolic process [GO:1903326]; negatively regulates tRNA metabolic process [GO:0006399] Also known as: down regulation of tRNA metabolic process, down regulation of tRNA metabolism, down-regulation of tRNA metabolic process, down-regulation of tRNA metabolism, downregulation of tRNA metabolic process, downregulation of tRNA metabolism, negative regulation of tRNA metabolism, inhibition of tRNA metabolic process, inhibition of tRNA metabolism Subtypes: negative regulation of tRNA catabolic process [GO:1902371], GO:2000236 Definition: Any process that stops, prevents or reduces the frequency, rate or extent of tRNA metabolic process. Sources: GOC:TermGenie, GOC:vw, GO_REF:0000058